{
  "gene": "UniProtKB:Q5TAP6",
  "gene_symbol": "UTP14C",
  "term_id": "GO:0032040",
  "gene_name": "U3 small nucleolar RNA-associated protein 14 homolog C",
  "term_label": "small-subunit processome"
}